{
  "term_id": "GO:0043025",
  "term_label": "neuronal cell body",
  "gene": "UniProtKB:Q53EL9",
  "gene_symbol": "SEZ6",
  "gene_name": "Seizure protein 6 homolog"
}